{
  "term_id": "GO:0030527",
  "gene": "UniProtKB:P68431",
  "gene_symbol": "H3C12",
  "gene_name": "Histone H3.1",
  "term_label": "structural constituent of chromatin"
}